meiotic M phase [GO:0051327] (biological process) Note: Note that this term should not be used for direct annotation. If you are trying to make an annotation to x phase, it is likely that the correct annotation is 'regulation of x/y phase transition' or to a process which occurs during the reported phase (i.e mitotic DNA replication for mitotic S-phase). To capture the phase when a specific location or process is observed, the phase term can be used in an annotation extension (PMID:24885854) applied to a cellular component term (with the relation exists_during) or a biological process term (with the relation happens_during). Relationships: is_a GO:0000279; is a type of meiotic cell cycle phase [GO:0098762] Sources: GOC:mtg_cell_cycle Definition: A cell cycle phase during which nuclear division occurs, and which is comprises the phases: prophase, metaphase, anaphase and telophase and occurs as part of a meiotic cell cycle. Also known as: M phase of meiotic cell cycle